{
  "term_label": "nucleolus",
  "gene_name": "28S rRNA (cytosine-C(5))-methyltransferase",
  "term_id": "GO:0005730",
  "gene_symbol": "NSUN5",
  "gene": "UniProtKB:Q96P11"
}